uracil oxygenase activity [GO:0052614] (molecular function) Relationships: is a type of oxidoreductase activity, acting on paired donors, with incorporation or reduction of molecular oxygen [GO:0016705] Also known as: pyrimidine oxygenase activity References: PMID:20369853, PMID:20400551 Sources: RHEA:31587 Definition: Catalysis of the reaction: FMNH2 + NADH + O2 + uracil = (Z)-3-ureidoacrylate + FMN + H+ + H2O + NAD+. Can also use thymine as a substrate.